{
  "term_id": "GO:0060326",
  "gene": "UniProtKB:Q30KR1",
  "gene_symbol": "DEFB109B",
  "term_label": "cell chemotaxis",
  "gene_name": "Putative beta-defensin 109B"
}